{
  "gene": "UniProtKB:Q5JSL3",
  "term_id": "UNKNOWN:0003",
  "term_label": "Unknown cellular component",
  "gene_symbol": "DOCK11",
  "gene_name": "Dedicator of cytokinesis protein 11"
}